positive regulation of protein localization to chromatin [GO:0120187] (biological process) References: PMID:20889714, PMID:29899453 Relationships: is a type of positive regulation of protein localization [GO:1903829]; is a type of regulation of protein localization to chromatin [GO:1905634]; positively regulates protein localization to chromatin [GO:0071168] Also known as: positive regulation of protein localisation to chromatin Definition: Any process that activates or increases the frequency, rate or extent of protein localization to chromatin.